{
  "term_id": "GO:0031012",
  "gene_name": "EGF-containing fibulin-like extracellular matrix protein 2",
  "term_label": "extracellular matrix",
  "gene": "UniProtKB:O95967",
  "gene_symbol": "EFEMP2"
}